meiotic G1 phase [GO:0051330] (biological process) Relationships: is a type of G1 phase [GO:0051318]; is part of GO:0051328 Note: Note that this term should not be used for direct annotation. If you are trying to make an annotation to x phase, it is likely that the correct annotation is 'regulation of x/y phase transition' or to a process which occurs during the reported phase (i.e mitotic DNA replication for mitotic S-phase). To capture the phase when a specific location or process is observed, the phase term can be used in an annotation extension (PMID:24885854) applied to a cellular component term (with the relation exists_during) or a biological process term (with the relation happens_during). Also known as: G1 phase of meiotic cell cycle Sources: GOC:mtg_cell_cycle Definition: The cell cycle 'gap' phase which is the interval between the completion of DNA segregation by meiosis and the beginning of DNA synthesis.